{
  "gene_symbol": "PCSK1",
  "gene": "UniProtKB:P29120",
  "term_id": "GO:0043005",
  "gene_name": "Neuroendocrine convertase 1",
  "term_label": "neuron projection"
}